{
  "term_label": "intracellular signal transduction",
  "gene_name": "Serine_threonine-protein kinase Sgk2",
  "gene": "UniProtKB:Q9HBY8",
  "gene_symbol": "SGK2",
  "term_id": "GO:0035556"
}